integrin alphaIIb-beta3 complex [GO:0070442] (cellular component) Definition: An integrin complex that comprises one alphaIIb subunit and one beta3 subunit. Also known as: alphaIIb-beta3 integrin complex, ITGA2B-ITGB3 complex References: PMID:12297042 Relationships: is a type of integrin complex [GO:0008305]